{
  "gene_symbol": "TTC17",
  "term_id": "GO:0005737",
  "term_label": "cytoplasm",
  "gene_name": "Tetratricopeptide repeat protein 17",
  "gene": "UniProtKB:Q96AE7"
}